myeloid cell development [GO:0061515] (biological process) Definition: The process whose specific outcome is the progression of a myeloid cell over time, from its formation to the mature structure. Sources: GOC:dph Relationships: is a type of hemopoiesis [GO:0030097]; is part of GO:0030099 Subtypes: microglia development [GO:0014005], megakaryocyte development [GO:0035855], osteoclast development [GO:0036035], GO:0048821